{
  "gene": "UniProtKB:Q8N9Z0",
  "term_label": "RNA polymerase II cis-regulatory region sequence-specific DNA binding",
  "gene_name": "Zinc finger protein 610",
  "term_id": "GO:0000978",
  "gene_symbol": "ZNF610"
}